{
  "gene_symbol": "MATN2",
  "gene": "UniProtKB:O00339",
  "gene_name": "Matrilin-2",
  "term_label": "extracellular matrix",
  "term_id": "GO:0031012"
}